glycine amidinotransferase activity [GO:0015068] (molecular function) Sources: RHEA:13201 Relationships: is a type of amidinotransferase activity [GO:0015067] Definition: Catalysis of the reaction: L-arginine + glycine = L-ornithine + guanidinoacetate. Also known as: L-arginine:glycine amidinotransferase activity, arginine-glycine amidinotransferase activity, arginine-glycine transamidinase activity, glycine transamidinase activity